{
  "gene": "UniProtKB:P62952",
  "term_id": "UNKNOWN:0001",
  "term_label": "Unknown molecular function",
  "gene_name": "Bladder cancer-associated protein",
  "gene_symbol": "BLCAP"
}